{
  "gene_symbol": "KIR2DL1",
  "gene": "UniProtKB:A0A191URJ7",
  "term_label": "immune response-inhibiting cell surface receptor signaling pathway",
  "term_id": "GO:0002767",
  "gene_name": "KIR2DL protein"
}